{
  "term_label": "neuronal cell body",
  "gene_symbol": "KNDC1",
  "term_id": "GO:0043025",
  "gene_name": "Kinase non-catalytic C-lobe domain-containing protein 1",
  "gene": "UniProtKB:Q76NI1"
}